{
  "term_id": "GO:0043123",
  "gene_symbol": "RIPK2",
  "gene": "UniProtKB:O43353",
  "term_label": "positive regulation of canonical NF-kappaB signal transduction",
  "gene_name": "Receptor-interacting serine_threonine-protein kinase 2"
}